{
  "term_id": "GO:0051427",
  "gene_symbol": "NPPC",
  "term_label": "hormone receptor binding",
  "gene_name": "C-type natriuretic peptide",
  "gene": "UniProtKB:P23582"
}